mesonephric capsule specification [GO:0061288] (biological process) Sources: GOC:mtg_kidney_jan10 Relationships: is a type of pattern specification involved in mesonephros development [GO:0061227]; is a type of renal capsule specification [GO:0072130]; is part of GO:0061287 Definition: The regionalization process in which the identity of the mesonephric capsule is specified. Identity is considered to be the aggregate of characteristics by which a structure is recognized.